{
  "term_id": "GO:0120044",
  "gene_symbol": "TPRN",
  "gene_name": "Taperin",
  "gene": "UniProtKB:Q4KMQ1",
  "term_label": "stereocilium base"
}